{
  "term_label": "negative regulation of sequestering of calcium ion",
  "term_id": "GO:0051283",
  "gene_name": "Annexin A6",
  "gene_symbol": "ANXA6",
  "gene": "UniProtKB:P08133"
}